{
  "gene_symbol": "SLCO1B1",
  "gene": "UniProtKB:Q9Y6L6",
  "term_id": "GO:0016323",
  "term_label": "basolateral plasma membrane",
  "gene_name": "Solute carrier organic anion transporter family member 1B1"
}